{
  "term_label": "ubiquitin-like ligase-substrate adaptor activity",
  "gene_symbol": "KLHL25",
  "gene_name": "Kelch-like protein 25",
  "term_id": "GO:1990756",
  "gene": "UniProtKB:Q9H0H3"
}